folic acid-containing compound catabolic process [GO:0009397] (biological process) Subtypes: 10-formyltetrahydrofolate catabolic process [GO:0009258], folic acid catabolic process [GO:0046657] Definition: The chemical reactions and pathways resulting in the breakdown of folic acid and its derivatives. Relationships: is a type of GO:0006760; is a type of modified amino acid catabolic process [GO:0042219]; is a type of pteridine-containing compound catabolic process [GO:0042560] Sources: GOC:ai Also known as: folate and derivative catabolic process, folate and derivative catabolism, folate-containing compound catabolic process, folate-containing compound catabolism, folic acid and derivative catabolic process, folic acid and derivative catabolism, folic acid-containing compound breakdown, folic acid-containing compound catabolism, folic acid-containing compound degradation, vitamin B9 and derivative catabolic process, vitamin B9 and derivative catabolism, vitamin M and derivative catabolic process, vitamin M and derivative catabolism